DNA-5-methylcytosine glycosylase activity [GO:1990053] (molecular function) References: PMID:23316050 Definition: Catalysis of the reaction: DNA containing 5-methylcytosine + H2O = DNA with abasic site + 5-methylcytosine. This reaction is the hydrolysis of DNA by cleavage of the N-C1' glycosidic bond between the DNA 5-methylcytosine and the deoxyribose sugar to remove the 5-methylcytosine, leaving an abasic site. Relationships: is a type of alkylbase DNA N-glycosylase activity [GO:0003905]